{
  "term_id": "GO:0047186",
  "gene_symbol": "CASD1",
  "term_label": "N-acetylneuraminate 9-O-acetyltransferase activity",
  "gene_name": "N-acetylneuraminate 9-O-acetyltransferase",
  "gene": "UniProtKB:Q96PB1"
}